{
  "gene": "UniProtKB:Q6MZZ7",
  "gene_symbol": "CAPN13",
  "term_id": "GO:0006508",
  "term_label": "proteolysis",
  "gene_name": "Calpain-13"
}